{
  "gene_symbol": "PJA1",
  "term_id": "GO:0005737",
  "term_label": "cytoplasm",
  "gene": "UniProtKB:Q8NG27",
  "gene_name": "E3 ubiquitin-protein ligase Praja-1"
}